{
  "term_label": "peptide cross-linking",
  "gene_symbol": "EPB42",
  "gene": "UniProtKB:P16452",
  "term_id": "GO:0018149",
  "gene_name": "Protein 4.2"
}